methylglyoxal catabolic process to lactate [GO:0061727] (biological process) Subtypes: methylglyoxal catabolic process to D-lactate via S-lactoyl-glutathione [GO:0019243], D-lactate biosynthetic process from methylglyoxal via (R)-lactaldehyde [GO:0019248] Relationships: is a type of lactate metabolic process [GO:0006089]; is a type of methylglyoxal catabolic process [GO:0051596] Definition: The chemical reactions and pathways resulting in the breakdown of methylglyoxal, CH3-CO-CHO, into lactate. References: PMID:2198020 Sources: GOC:dph